ABC-type 3',5'-cyclic GMP transmembrane transporter activity [GO:1905948] (molecular function) Definition: Enables the transfer of a solute or solutes from one side of a membrane to the other according to the reaction: ATP + H2O + 3',5'-cyclic GMP(in) = ADP + phosphate + 3',5'-cyclic GMP(out). Also known as: 3',5'-cyclic GMP transmembrane-transporting ATPase activity, ATP-dependent 3',5'-cyclic GMP transmembrane transporter activity, ATPase-coupled cGMP transmembrane transporter activity, ATPase-coupled 3',5'-cyclic GMP transmembrane transporter activity Relationships: is a type of guanine nucleotide transmembrane transporter activity [GO:0001409]; is_a purine ribonucleotide transmembrane transporter activity [GO:0005346]; is a type of ABC-type transporter activity [GO:0140359] References: PMID:18310115 Sources: GOC:TermGenie, GO_REF:0000070